neural plate anterior/posterior regionalization [GO:0021999] (biological process) Sources: GOC:cls, GOC:dgh, GOC:dph, GOC:jid, GO_REF:0000021 Also known as: neural plate anterior/posterior pattern formation Relationships: is a type of GO:0009952; is a type of neural plate regionalization [GO:0060897] Definition: The process that regulates the coordinated growth and differentiation that establishes the non-random anterior-posterior spatial arrangement of the neural plate.